{
  "term_label": "cytoplasm",
  "gene_symbol": "STMN1",
  "gene_name": "Stathmin",
  "term_id": "GO:0005737",
  "gene": "UniProtKB:P16949"
}